fonsecin biosynthetic process [GO:1900769] (biological process) Relationships: is a type of GO:0030639; is a type of GO:0046165; is a type of phenol-containing compound biosynthetic process [GO:0046189]; is a type of naphtho-gamma-pyrone biosynthetic process [GO:1900787]; is a type of GO:1901503 Also known as: fonsecin anabolism, fonsecin biosynthesis, fonsecin formation, fonsecin synthesis Definition: The chemical reactions and pathways resulting in the formation of fonsecin. Sources: GOC:TermGenie, GOC:di